{
  "gene_symbol": "CDC16",
  "gene": "UniProtKB:Q13042",
  "gene_name": "Cell division cycle protein 16 homolog",
  "term_label": "positive regulation of mitotic metaphase/anaphase transition",
  "term_id": "GO:0045842"
}